{
  "term_label": "spliceosomal complex",
  "gene": "UniProtKB:Q15696",
  "gene_symbol": "ZRSR2",
  "term_id": "GO:0005681",
  "gene_name": "U2 small nuclear ribonucleoprotein auxiliary factor 35 kDa subunit-related protein 2"
}